{
  "gene": "UniProtKB:P0DKL9",
  "term_label": "Unknown molecular function",
  "gene_name": "ARL14 effector protein-like",
  "term_id": "UNKNOWN:0001",
  "gene_symbol": "ARL14EPL"
}